{
  "gene": "UniProtKB:Q9H7B4",
  "term_label": "histone H3K36 dimethyltransferase activity",
  "gene_symbol": "SMYD3",
  "term_id": "GO:0140954",
  "gene_name": "Histone-lysine N-methyltransferase SMYD3"
}